IMP metabolic process [GO:0046040] (biological process) Definition: The chemical reactions and pathways involving IMP, inosine monophosphate. Also known as: IMP metabolism Relationships: is a type of purine ribonucleotide metabolic process [GO:0009150]; is a type of purine ribonucleoside monophosphate metabolic process [GO:0009167] Sources: GOC:go_curators Subtypes: IMP biosynthetic process [GO:0006188], GMP catabolic process to IMP [GO:0006201], GO:0006204